{
  "gene_symbol": "RESP18",
  "gene_name": "Regulated endocrine-specific protein 18",
  "gene": "UniProtKB:Q5W5W9",
  "term_id": "UNKNOWN:0001",
  "term_label": "Unknown molecular function"
}